5-amino-1-ribofuranosylimidazole-4-carboxamide transmembrane transport [GO:1903088] (biological process) Definition: The process in which 5-amino-1-ribofuranosylimidazole-4-carboxamide is transported across a membrane. References: PMID:24778186 Sources: GOC:TermGenie, GO_REF:0000069 Relationships: is a type of amide transport [GO:0042886]; is a type of GO:0045117; is a type of carbohydrate derivative transport [GO:1901264]